{
  "gene_symbol": "MUCL1",
  "term_id": "UNKNOWN:0003",
  "term_label": "Unknown cellular component",
  "gene": "UniProtKB:Q96DR8",
  "gene_name": "Mucin-like protein 1"
}